{
  "term_label": "fatty acid biosynthetic process",
  "gene_symbol": "PNLIPRP1",
  "term_id": "GO:0006633",
  "gene_name": "Inactive pancreatic lipase-related protein 1",
  "gene": "UniProtKB:P54315"
}